{
  "gene": "UniProtKB:P10619",
  "gene_symbol": "CTSA",
  "term_label": "serine-type carboxypeptidase activity",
  "term_id": "GO:0004185",
  "gene_name": "Lysosomal protective protein"
}